{
  "gene_name": "Heterogeneous nuclear ribonucleoprotein H",
  "gene": "UniProtKB:P31943",
  "term_id": "GO:0043484",
  "gene_symbol": "HNRNPH1",
  "term_label": "regulation of RNA splicing"
}